{
  "gene_name": "Metastasis-associated protein MTA1",
  "term_label": "negative regulation of transcription by RNA polymerase II",
  "gene": "UniProtKB:Q13330",
  "term_id": "GO:0000122",
  "gene_symbol": "MTA1"
}